{
  "gene_name": "Mitogen-activated protein kinase-binding protein 1",
  "term_id": "GO:0043124",
  "gene_symbol": "MAPKBP1",
  "gene": "UniProtKB:O60336",
  "term_label": "negative regulation of canonical NF-kappaB signal transduction"
}